{
  "gene_name": "Nucleolar protein 9",
  "term_id": "GO:0000480",
  "term_label": "endonucleolytic cleavage in 5'-ETS of tricistronic rRNA transcript (SSU-rRNA, 5.8S rRNA, LSU-rRNA)",
  "gene_symbol": "NOP9",
  "gene": "UniProtKB:Q86U38"
}